{
  "gene": "UniProtKB:Q9HD90",
  "gene_symbol": "NEUROD4",
  "term_label": "axon development",
  "term_id": "GO:0061564",
  "gene_name": "Neurogenic differentiation factor 4"
}